{
  "term_id": "GO:0000786",
  "gene_name": "Histone H2B type 1-C_E_F_G_I",
  "gene_symbol": "H2BC10",
  "term_label": "nucleosome",
  "gene": "UniProtKB:P62807"
}